{
  "term_id": "GO:0016287",
  "term_label": "glycerone-phosphate O-acyltransferase activity",
  "gene_name": "Dihydroxyacetone phosphate acyltransferase",
  "gene_symbol": "GNPAT",
  "gene": "UniProtKB:O15228"
}